{
  "term_id": "UNKNOWN:0001",
  "gene_name": "Protein GDF5-AS1, mitochondrial",
  "term_label": "Unknown molecular function",
  "gene": "UniProtKB:Q5U4N7",
  "gene_symbol": "GDF5-AS1"
}